{
  "gene_symbol": "EFCAB8",
  "term_label": "Unknown cellular component",
  "term_id": "UNKNOWN:0003",
  "gene": "UniProtKB:A8MWE9",
  "gene_name": "EF-hand calcium-binding domain-containing protein 8"
}